positive regulation of opsonization [GO:1903028] (BP) Also known as: up regulation of opsonization, up-regulation of opsonization, upregulation of opsonization, activation of opsonization Relationships: is a type of positive regulation of immune effector process [GO:0002699]; is a type of GO:0050766; is a type of regulation of opsonization [GO:1903027]; positively regulates GO:0008228 Definition: Any process that activates or increases the frequency, rate or extent of opsonization. References: PMID:22333221 Sources: GOC:BHF, GOC:TermGenie, GOC:rl, GO_REF:0000058